{
  "gene": "UniProtKB:A6NHL2",
  "term_id": "GO:0005874",
  "term_label": "microtubule",
  "gene_name": "Tubulin alpha chain-like 3",
  "gene_symbol": "TUBAL3"
}